{
  "term_id": "GO:0031838",
  "gene_symbol": "HBG1",
  "gene_name": "Hemoglobin subunit gamma-1",
  "term_label": "haptoglobin-hemoglobin complex",
  "gene": "UniProtKB:P69891"
}